{
  "term_id": "GO:0005634",
  "term_label": "nucleus",
  "gene_name": "Period circadian protein homolog 1",
  "gene_symbol": "PER1",
  "gene": "UniProtKB:O15534"
}